{
  "gene_name": "HLA class II histocompatibility antigen, DR beta 5 chain",
  "gene": "UniProtKB:Q30154",
  "term_id": "GO:0031902",
  "gene_symbol": "HLA-DRB5",
  "term_label": "late endosome membrane"
}